{
  "gene_symbol": "IER3",
  "term_label": "Unknown molecular function",
  "term_id": "UNKNOWN:0001",
  "gene": "UniProtKB:P46695",
  "gene_name": "Radiation-inducible immediate-early gene IEX-1"
}